regulation of beta-catenin-TCF complex assembly [GO:1904863] (biological process) Definition: Any process that modulates the frequency, rate or extent of beta-catenin-TCF complex assembly. Sources: GOC:PARL, GOC:TermGenie, GOC:bf, GO_REF:0000058 Also known as: regulation of beta-catenin-TCF complex formation, regulation of beta-catenin/LEF complex assembly, regulation of beta-catenin/LEF complex formation, regulation of beta-catenin/T-cell factor complex assembly, regulation of beta-catenin/T-cell factor complex formation, regulation of beta-catenin/lymphoid enhancer binding factor complex assembly, regulation of beta-catenin/lymphoid enhancer binding factor complex formation Relationships: is a type of regulation of protein-containing complex assembly [GO:0043254]; RO_0002211 beta-catenin-TCF complex assembly [GO:1904837] Subtypes: GO:1904864, GO:1904865